{
  "gene_symbol": "PRSS1",
  "gene": "UniProtKB:P07477",
  "term_id": "GO:0006508",
  "gene_name": "Serine protease 1",
  "term_label": "proteolysis"
}